{
  "gene_name": "Pancreatic triacylglycerol lipase",
  "gene_symbol": "PNLIP",
  "term_label": "extracellular space",
  "term_id": "GO:0005615",
  "gene": "UniProtKB:P16233"
}